{
  "term_id": "UNKNOWN:0002",
  "term_label": "Unknown biological process",
  "gene": "UniProtKB:A6NLX3",
  "gene_symbol": "SPDYE4",
  "gene_name": "Speedy protein E4"
}